{
  "gene_symbol": "PLEKHG2",
  "gene_name": "Pleckstrin homology domain-containing family G member 2",
  "term_label": "small GTPase binding",
  "term_id": "GO:0031267",
  "gene": "UniProtKB:Q9H7P9"
}